{
  "term_label": "Unknown cellular component",
  "gene_name": "Uncharacterized protein C4orf45",
  "term_id": "UNKNOWN:0003",
  "gene_symbol": "C4orf45",
  "gene": "UniProtKB:Q96LM5"
}